{
  "gene_symbol": "NR2F2",
  "term_label": "negative regulation of transcription by RNA polymerase II",
  "gene_name": "COUP transcription factor 2",
  "term_id": "GO:0000122",
  "gene": "UniProtKB:P24468"
}